{
  "term_label": "DNA-binding transcription repressor activity, RNA polymerase II-specific",
  "gene_symbol": "SNAI1",
  "gene": "UniProtKB:O95863",
  "term_id": "GO:0001227",
  "gene_name": "Zinc finger protein SNAI1"
}